{
  "gene_name": "ATP-binding cassette sub-family A member 2",
  "gene": "UniProtKB:Q9BZC7",
  "term_id": "GO:0006869",
  "term_label": "lipid transport",
  "gene_symbol": "ABCA2"
}